{
  "gene": "UniProtKB:P62333",
  "gene_symbol": "PSMC6",
  "term_id": "GO:0045899",
  "gene_name": "26S proteasome regulatory subunit 10B",
  "term_label": "positive regulation of RNA polymerase II transcription preinitiation complex assembly"
}